6-phosphofructokinase activity [GO:0003872] (molecular function) Also known as: phosphohexokinase activity, 6-phosphofructokinase reduction, 6-phosphofructose 1-kinase activity, ATP-dependent phosphofructokinase activity, ATP:D-fructose-6-phosphate 1-phosphotransferase activity, D-fructose-6-phosphate 1-phosphotransferase activity, PFK, fructose 6-phosphate kinase activity, fructose 6-phosphokinase activity, nucleotide triphosphate-dependent phosphofructokinase activity, phospho-1,6-fructokinase activity, phosphofructokinase (phosphorylating), phosphofructokinase I activity Relationships: is a type of GO:0008443; is part of glycolytic process through fructose-6-phosphate [GO:0061615] Sources: EC:2.7.1.11 Definition: Catalysis of the reaction: ATP + D-fructose-6-phosphate = ADP + D-fructose 1,6-bisphosphate.